ferroxidase complex [GO:1905862] (cellular component) References: PMID:16522632 Sources: GOC:TermGenie, GOC:bhm, GO_REF:0000088 Note: An example of this is FET3 in Saccharomyces cerevisiae (P38993) in PMID:16522632 (inferred from direct assay). Relationships: is_a oxidoreductase complex [GO:1990204] Definition: A protein complex which is capable of ferroxidase activity. Subtypes: high-affinity iron permease complex [GO:0033573], high-affinity iron exporter complex [GO:0061841]